{
  "term_id": "GO:0005634",
  "gene": "UniProtKB:Q9UIS9",
  "gene_symbol": "MBD1",
  "gene_name": "Methyl-CpG-binding domain protein 1",
  "term_label": "nucleus"
}